{
  "gene": "UniProtKB:O94955",
  "term_id": "GO:0005737",
  "term_label": "cytoplasm",
  "gene_name": "Rho-related BTB domain-containing protein 3",
  "gene_symbol": "RHOBTB3"
}